mitochondrial translation [GO:0032543] (biological process) Relationships: is a type of translation [GO:0006412]; is part of mitochondrial gene expression [GO:0140053]; occurs in mitochondrion [GO:0005739] Regulation: regulated by regulation of mitochondrial translation [GO:0070129]; negatively regulated by negative regulation of mitochondrial translation [GO:0070130]; positively regulated by GO:0070131 Sources: GOC:go_curators Definition: The chemical reactions and pathways resulting in the formation of a protein in a mitochondrion. This is a ribosome-mediated process in which the information in messenger RNA (mRNA) is used to specify the sequence of amino acids in the protein; the mitochondrion has its own ribosomes and transfer RNAs, and uses a genetic code that differs from the nuclear code. Also known as: mitochondrial protein anabolism, mitochondrial protein biosynthesis, mitochondrial protein formation, mitochondrial protein synthesis, mitochondrial protein translation